regulation of dendritic spine morphogenesis [GO:0061001] (biological process) Definition: Any process that modulates the rate, frequency, or extent of dendritic spine morphogenesis, the process in which the anatomical structures of a dendritic spine are generated and organized. A dendritic spine is a protrusion from a dendrite and a specialized subcellular compartment involved in synaptic transmission. Sources: GOC:dph Subtypes: negative regulation of dendritic spine morphogenesis [GO:0061002], positive regulation of dendritic spine morphogenesis [GO:0061003] Relationships: is a type of regulation of neuron projection development [GO:0010975]; is a type of regulation of anatomical structure morphogenesis [GO:0022603]; is a type of regulation of postsynapse organization [GO:0099175]; regulates dendritic spine morphogenesis [GO:0060997]